{
  "gene_name": "Reticulon-3",
  "gene": "UniProtKB:O95197",
  "term_label": "endoplasmic reticulum tubular network membrane organization",
  "gene_symbol": "RTN3",
  "term_id": "GO:1990809"
}